{
  "gene": "UniProtKB:O14513",
  "term_id": "GO:0007019",
  "gene_symbol": "NCKAP5",
  "gene_name": "Nck-associated protein 5",
  "term_label": "microtubule depolymerization"
}